{
  "gene_name": "Hepatocyte nuclear factor 6",
  "term_label": "DNA-binding transcription factor activity, RNA polymerase II-specific",
  "gene_symbol": "ONECUT1",
  "gene": "UniProtKB:Q9UBC0",
  "term_id": "GO:0000981"
}